{
  "gene": "UniProtKB:Q6UX98",
  "gene_symbol": "ZDHHC24",
  "term_label": "endoplasmic reticulum",
  "gene_name": "Probable palmitoyltransferase ZDHHC24",
  "term_id": "GO:0005783"
}